interleukin-23 complex [GO:0070743] (cellular component) Note: Note that this heterodimeric cytokine utilizes the same beta subunit as IL-12. Also known as: IL-23 complex, IL12B, IL23A, p19, p40 Definition: A protein complex that is composed of an interleukin-23 alpha (p19, product of the IL23A gene) and an interleukin-12 beta (p40, product of the IL12B gene) subunit and is secreted into the extracellular space. References: PMID:11114383, PMID:15999093 Sources: GOC:add Relationships: is_a GO:0032991; is part of extracellular space [GO:0005615]